{
  "gene_symbol": "PSTPIP2",
  "gene": "UniProtKB:Q9H939",
  "term_id": "GO:0005737",
  "term_label": "cytoplasm",
  "gene_name": "Proline-serine-threonine phosphatase-interacting protein 2"
}